chromatin-templated microtubule nucleation [GO:0090223] (biological process) Sources: GOC:ascb_2009, GOC:dph, GOC:tb Definition: The 'de novo' formation of a microtubule, in which tubulin heterodimers form metastable oligomeric aggregates from chromatin. Relationships: is a type of GO:0007020